{
  "term_id": "GO:0070971",
  "gene": "UniProtKB:Q9NR31",
  "gene_symbol": "SAR1A",
  "gene_name": "GTP-binding protein SAR1a",
  "term_label": "endoplasmic reticulum exit site"
}